{
  "term_id": "GO:0006357",
  "term_label": "regulation of transcription by RNA polymerase II",
  "gene_symbol": "POU1F1",
  "gene": "UniProtKB:P28069",
  "gene_name": "Pituitary-specific positive transcription factor 1"
}